mitochondrial tRNA processing [GO:0090646] (biological process) Sources: GOC:vw Definition: The process in which a pre-tRNA molecule is converted to a mature tRNA, ready for addition of an aminoacyl group, in the mitochondrion. Subtypes: mitochondrial tRNA modification [GO:0070900], mitochondrial tRNA 5'-end processing [GO:0097745], mitochondrial tRNA 3'-end processing [GO:1990180] Relationships: is a type of mitochondrial RNA metabolic process [GO:0000959]; is a type of mitochondrial RNA processing [GO:0000963]; is a type of tRNA processing [GO:0008033]